{
  "gene_symbol": "HLA-E",
  "term_id": "GO:0009897",
  "gene_name": "HLA class I histocompatibility antigen, alpha chain E",
  "gene": "UniProtKB:P13747",
  "term_label": "external side of plasma membrane"
}